citryl-CoA lyase activity [GO:0008816] (molecular function) Definition: Catalysis of the reaction: (3S)-citryl-CoA = acetyl-CoA + oxaloacetate. Also known as: (3S)-citryl-CoA oxaloacetate-lyase (acetyl-CoA-forming), (3S)-citryl-CoA oxaloacetate-lyase activity Sources: EC:4.1.3.34 Relationships: is_a GO:0016833